{
  "term_id": "GO:0015629",
  "gene_symbol": "CALD1",
  "gene_name": "Caldesmon",
  "term_label": "actin cytoskeleton",
  "gene": "UniProtKB:Q05682"
}